{
  "gene_symbol": "IGKV2D-30",
  "term_label": "Unknown molecular function",
  "gene_name": "Immunoglobulin kappa variable 2D-30",
  "gene": "UniProtKB:A0A075B6S6",
  "term_id": "UNKNOWN:0001"
}